{
  "gene_symbol": "RBM14",
  "gene": "UniProtKB:Q96PK6",
  "term_label": "mRNA binding",
  "gene_name": "RNA-binding protein 14",
  "term_id": "GO:0003729"
}